synaptic vesicle fusion to presynaptic active zone membrane [GO:0031629] (biological process) Regulation: regulated by GO:0031630; negatively regulated by negative regulation of synaptic vesicle fusion to presynaptic active zone membrane [GO:0031631]; positively regulated by positive regulation of synaptic vesicle fusion to presynaptic active zone membrane [GO:0031632] Definition: Fusion of the membrane of a synaptic vesicle with the presynaptic active zone membrane, thereby releasing its cargo neurotransmitters into the synaptic cleft. References: PMID:18618940 Sources: GOC:aruk, GOC:bc, ISBN:0071120009 Also known as: synaptic vesicle fusion, synaptic vesicle fusion to pre-synaptic membrane, synaptic vesicle fusion to presynaptic membrane Relationships: is a type of synaptic vesicle membrane organization [GO:0048499]; is a type of GO:0099500; is part of synaptic vesicle exocytosis [GO:0016079]